{
  "gene_name": "Zinc transporter SLC39A7",
  "term_id": "UNKNOWN:0003",
  "gene_symbol": "SLC39A7",
  "gene": "UniProtKB:Q92504",
  "term_label": "Unknown cellular component"
}